{
  "gene_symbol": "IGHA2",
  "term_id": "GO:0019731",
  "term_label": "antibacterial humoral response",
  "gene": "UniProtKB:P01877",
  "gene_name": "Immunoglobulin heavy constant alpha 2"
}